{
  "term_id": "GO:0036376",
  "gene_name": "Sodium_potassium-transporting ATPase subunit beta-1",
  "gene_symbol": "ATP1B1",
  "gene": "UniProtKB:P05026",
  "term_label": "sodium ion export across plasma membrane"
}